{
  "term_id": "GO:0005737",
  "gene_symbol": "AZIN2",
  "gene_name": "Antizyme inhibitor 2",
  "gene": "UniProtKB:Q96A70",
  "term_label": "cytoplasm"
}